{
  "term_id": "UNKNOWN:0003",
  "term_label": "Unknown cellular component",
  "gene": "UniProtKB:Q9P242",
  "gene_symbol": "NYAP2",
  "gene_name": "Neuronal tyrosine-phosphorylated phosphoinositide-3-kinase adapter 2"
}